{
  "term_id": "GO:0003727",
  "gene_symbol": "STRBP",
  "gene_name": "Spermatid perinuclear RNA-binding protein",
  "gene": "UniProtKB:Q96SI9",
  "term_label": "single-stranded RNA binding"
}